fatty acid homeostasis [GO:0055089] (biological process) Definition: Any process involved in the maintenance of an internal steady state of fatty acid within an organism or cell. Relationships: is a type of lipid homeostasis [GO:0055088] Sources: GOC:BHF, GOC:rl